astrocyte projection [GO:0097449] (cellular component) Relationships: is a type of GO:0097386 Definition: A prolongation or process extending from the soma of an astrocyte and wrapping around neurons. Also known as: astrocyte process, peripheral astrocyte process, vellous process Sources: NIF_Subcellular:sao1630537580 Subtypes: GO:0097450